{
  "gene_name": "Tripartite motif-containing protein 10",
  "gene": "UniProtKB:Q9UDY6",
  "term_id": "GO:0005737",
  "gene_symbol": "TRIM10",
  "term_label": "cytoplasm"
}